{
  "term_id": "GO:0050770",
  "gene_name": "Serine_threonine-protein kinase PAK 1",
  "term_label": "regulation of axonogenesis",
  "gene_symbol": "PAK1",
  "gene": "UniProtKB:Q13153"
}